{
  "term_label": "Unknown biological process",
  "gene_symbol": "LINC00862",
  "gene": "UniProtKB:A6NCI5",
  "gene_name": "Putative transmembrane protein encoded by LINC00862",
  "term_id": "UNKNOWN:0002"
}